{
  "gene_symbol": "PDGFRB",
  "term_label": "positive regulation of cell population proliferation",
  "gene": "UniProtKB:P09619",
  "gene_name": "Platelet-derived growth factor receptor beta",
  "term_id": "GO:0008284"
}